{
  "term_id": "GO:0031369",
  "gene_symbol": "EIF3C",
  "gene": "UniProtKB:Q99613",
  "term_label": "translation initiation factor binding",
  "gene_name": "Eukaryotic translation initiation factor 3 subunit C"
}